embryonic lung development [GO:1990401] (biological process) Definition: The process occurring during the embryonic phase whose specific outcome is the progression of the lung over time, from its formation to the mature structure. References: PMID:24785085 Relationships: is a type of GO:0048568